{
  "gene_symbol": "RUNX2",
  "term_id": "GO:0030097",
  "gene_name": "Runt-related transcription factor 2",
  "term_label": "hemopoiesis",
  "gene": "UniProtKB:Q13950"
}